{
  "gene_name": "Ras-related C3 botulinum toxin substrate 3",
  "gene": "UniProtKB:P60763",
  "term_label": "GTPase activity",
  "term_id": "GO:0003924",
  "gene_symbol": "RAC3"
}